{
  "gene_name": "Basic leucine zipper transcriptional factor ATF-like",
  "term_id": "GO:0000978",
  "term_label": "RNA polymerase II cis-regulatory region sequence-specific DNA binding",
  "gene_symbol": "BATF",
  "gene": "UniProtKB:Q16520"
}